anaerobic phenol-containing compound metabolic process [GO:0042215] (biological process) Relationships: is a type of phenol-containing compound metabolic process [GO:0018958] Definition: The chemical reactions and pathways involving a phenol, any compound containing one or more hydroxyl groups directly attached to an aromatic carbon ring, in the absence of oxygen. References: PMID:12697029 Subtypes: anaerobic phenol-containing compound biosynthetic process [GO:0046192], anaerobic phenol-containing compound catabolic process [GO:0046193] Also known as: anaerobic phenol-containing compound metabolism